{
  "gene": "UniProtKB:Q8IVK1",
  "term_label": "Unknown molecular function",
  "gene_name": "Putative glycosylation-dependent cell adhesion molecule 1",
  "term_id": "UNKNOWN:0001",
  "gene_symbol": "GLYCAM1"
}